{
  "term_label": "basolateral plasma membrane",
  "gene_symbol": "PDZD11",
  "gene": "UniProtKB:Q5EBL8",
  "term_id": "GO:0016323",
  "gene_name": "PDZ domain-containing protein 11"
}